{
  "gene": "UniProtKB:Q8TC29",
  "term_id": "GO:0005516",
  "term_label": "calmodulin binding",
  "gene_name": "Enkurin",
  "gene_symbol": "ENKUR"
}